{
  "term_label": "sperm axoneme assembly",
  "gene_name": "Cilia- and flagella-associated protein 43",
  "gene_symbol": "CFAP43",
  "term_id": "GO:0007288",
  "gene": "UniProtKB:Q8NDM7"
}